{
  "term_id": "GO:0005737",
  "term_label": "cytoplasm",
  "gene_name": "Guanine nucleotide-binding protein subunit beta-5",
  "gene_symbol": "GNB5",
  "gene": "UniProtKB:O14775"
}